{
  "term_label": "regulation of transcription by RNA polymerase II",
  "gene_symbol": "FOXP1",
  "term_id": "GO:0006357",
  "gene": "UniProtKB:Q9H334",
  "gene_name": "Forkhead box protein P1"
}